{
  "gene": "UniProtKB:Q8TE77",
  "gene_symbol": "SSH3",
  "gene_name": "Protein phosphatase Slingshot homolog 3",
  "term_id": "GO:0005737",
  "term_label": "cytoplasm"
}